{
  "gene_name": "Peptidyl-prolyl cis-trans isomerase FKBP2",
  "term_id": "UNKNOWN:0002",
  "gene": "UniProtKB:P26885",
  "term_label": "Unknown biological process",
  "gene_symbol": "FKBP2"
}